{
  "gene_name": "Grancalcin",
  "term_id": "UNKNOWN:0003",
  "gene": "UniProtKB:P28676",
  "gene_symbol": "GCA",
  "term_label": "Unknown cellular component"
}